regulation of proteasomal protein catabolic process [GO:0061136] (biological process) Subtypes: regulation of proteasomal ubiquitin-dependent protein catabolic process [GO:0032434], negative regulation of proteasomal protein catabolic process [GO:1901799], positive regulation of proteasomal protein catabolic process [GO:1901800], regulation of ERAD pathway [GO:1904292] Relationships: is a type of regulation of protein catabolic process [GO:0042176]; is a type of GO:1903050; regulates proteasomal protein catabolic process [GO:0010498] Definition: Any process that modulates the rate, frequency, or extent of the chemical reactions and pathways resulting in the breakdown of a protein or peptide by hydrolysis of its peptide bonds that is mediated by the proteasome. Sources: GOC:dph, GOC:tb